{
  "gene_symbol": "HTT",
  "gene": "UniProtKB:P42858",
  "term_id": "GO:0022008",
  "gene_name": "Huntingtin",
  "term_label": "neurogenesis"
}